{
  "gene": "UniProtKB:P22557",
  "term_label": "5-aminolevulinate synthase activity",
  "gene_name": "5-aminolevulinate synthase, erythroid-specific, mitochondrial",
  "term_id": "GO:0003870",
  "gene_symbol": "ALAS2"
}